{
  "gene": "UniProtKB:O43435",
  "term_id": "GO:0001708",
  "gene_name": "T-box transcription factor TBX1",
  "gene_symbol": "TBX1",
  "term_label": "cell fate specification"
}